{
  "term_label": "Unknown cellular component",
  "term_id": "UNKNOWN:0003",
  "gene_symbol": "TMEM161B",
  "gene": "UniProtKB:Q8NDZ6",
  "gene_name": "Transmembrane protein 161B"
}